{
  "gene_symbol": "S1PR5",
  "term_label": "cytoplasm",
  "gene_name": "Sphingosine 1-phosphate receptor 5",
  "gene": "UniProtKB:Q9H228",
  "term_id": "GO:0005737"
}